{
  "gene_name": "1-acyl-sn-glycerol-3-phosphate acyltransferase epsilon",
  "term_label": "mitochondrion",
  "gene_symbol": "AGPAT5",
  "term_id": "GO:0005739",
  "gene": "UniProtKB:Q9NUQ2"
}